{
  "term_id": "GO:0042059",
  "term_label": "negative regulation of epidermal growth factor receptor signaling pathway",
  "gene": "UniProtKB:O43597",
  "gene_name": "Protein sprouty homolog 2",
  "gene_symbol": "SPRY2"
}